positive regulation of response to stimulus [GO:0048584] (BP) Relationships: is a type of positive regulation of biological process [GO:0048518]; is a type of GO:0048583; positively regulates response to stimulus [GO:0050896] Note: Note that this term is in the subset of terms that should not be used for direct gene product annotation. Instead, select a child term or, if no appropriate child term exists, please request a new term. Direct annotations to this term may be amended during annotation QC. Subtypes: GO:0002833, positive regulation of signal transduction [GO:0009967], positive regulation of vernalization response [GO:0010220], positive regulation of muscle adaptation [GO:0014744], positive regulation of defense response [GO:0031349], positive regulation of response to external stimulus [GO:0032103], positive regulation of response to nutrient levels [GO:0032109], positive regulation of DNA repair [GO:0045739], positive regulation of establishment of competence for transformation [GO:0045809], positive regulation of short-day photoperiodism, flowering [GO:0048576], GO:0048578, GO:0050778, positive regulation of response to cytokine stimulus [GO:0060760], positive regulation of neuron projection regeneration [GO:0070572], positive regulation of thermomorphogenesis [GO:0140922], positive regulation of cellular response to heat [GO:1900036], positive regulation of cellular response to hypoxia [GO:1900039], positive regulation of cellular response to insulin stimulus [GO:1900078], GO:1900433, GO:1900439, positive regulation of response to pullulan [GO:1900520], positive regulation of response to amylopectin [GO:1900523], positive regulation of filamentous growth of a population of unicellular organisms in response to pH [GO:1900743], positive regulation of response to salt stress [GO:1901002], GO:1901421, positive regulation of response to cycloalkane [GO:1901433], GO:1901444, positive regulation of response to benzene [GO:1901453], GO:1901456, positive regulation of response to acetate [GO:1901459], positive regulation of response to formic acid [GO:1901462], positive regulation of shade avoidance [GO:1902448], positive regulation of response to water deprivation [GO:1902584], GO:1902884, positive regulation of response to wounding [GO:1903036], positive regulation of fear response [GO:1903367], positive regulation of cellular response to transforming growth factor beta stimulus [GO:1903846], positive regulation of stress response to copper ion [GO:1903855], positive regulation of error-prone translesion synthesis [GO:1904333], positive regulation of telomere maintenance in response to DNA damage [GO:1904507], positive regulation of xenobiotic detoxification by transmembrane export across the plasma membrane [GO:1905701], positive regulation of cellular response to manganese ion [GO:1905804], positive regulation of cellular response to oxidopamine [GO:1905848], positive regulation of cellular response to very-low-density lipoprotein particle stimulus [GO:1905889], positive regulation of response to endoplasmic reticulum stress [GO:1905898], positive regulation of response to calcium ion [GO:1905947], GO:2000306, positive regulation of cellular response to X-ray [GO:2000685], positive regulation of detection of glucose [GO:2000972], positive regulation of response to drug [GO:2001025], positive regulation of cellular response to hepatocyte growth factor stimulus [GO:2001114], GO:2001230 Sources: GOC:jid Definition: Any process that activates, maintains or increases the rate of a response to a stimulus. Response to stimulus is a change in state or activity of a cell or an organism (in terms of movement, secretion, enzyme production, gene expression, etc.) as a result of a stimulus. Also known as: up regulation of response to stimulus, up-regulation of response to stimulus, upregulation of response to stimulus, activation of response to stimulus, stimulation of response to stimulus